negative regulation of amino acid biosynthetic process [GO:2000283] (biological process) Subtypes: GO:0062133, GO:0120214, GO:1901711, GO:1902006, GO:1902987, GO:1903196, negative regulation of citrulline biosynthetic process [GO:1903249], negative regulation of L-leucine biosynthetic process [GO:2001277] Sources: GOC:obol Relationships: is a type of negative regulation of biosynthetic process [GO:0009890]; is a type of GO:0045763; is a type of regulation of amino acid biosynthetic process [GO:2000282]; negatively regulates amino acid biosynthetic process [GO:0008652] Definition: Any process that stops, prevents or reduces the frequency, rate or extent of an amino acid biosynthetic process. Also known as: negative regulation of amino acid anabolism, negative regulation of amino acid biosynthesis, negative regulation of amino acid formation, negative regulation of amino acid synthesis, negative regulation of cellular amino acid biosynthetic process